{
  "term_id": "GO:0004984",
  "gene": "UniProtKB:Q8NGH9",
  "gene_name": "Olfactory receptor 52E4",
  "gene_symbol": "OR52E4",
  "term_label": "olfactory receptor activity"
}